{
  "gene": "UniProtKB:Q3LI83",
  "gene_symbol": "KRTAP24-1",
  "term_id": "UNKNOWN:0001",
  "term_label": "Unknown molecular function",
  "gene_name": "Keratin-associated protein 24-1"
}